{
  "term_label": "Unknown biological process",
  "gene_name": "Olfactory receptor 4K3",
  "gene": "UniProtKB:Q96R72",
  "gene_symbol": "OR4K3",
  "term_id": "UNKNOWN:0002"
}